positive regulation of cholesterol metabolic process [GO:0090205] (biological process) Subtypes: positive regulation of cholesterol biosynthetic process [GO:0045542] Definition: Any process that increases the rate, frequency, or extent of cholesterol metabolism, the chemical reactions and pathways involving cholesterol, cholest-5-en-3 beta-ol, the principal sterol of vertebrates and the precursor of many steroids, including bile acids and steroid hormones. Relationships: is a type of positive regulation of steroid metabolic process [GO:0045940]; is_a GO:0062013; is_a GO:0090181; positively regulates cholesterol metabolic process [GO:0008203] Sources: GOC:dph, GOC:sl, GOC:tb